{
  "gene": "UniProtKB:Q8IXN7",
  "term_id": "GO:0005737",
  "gene_symbol": "RIMKLA",
  "term_label": "cytoplasm",
  "gene_name": "N-acetylaspartylglutamate synthase A"
}